{
  "gene_name": "RNA binding protein fox-1 homolog 2",
  "term_id": "GO:0003729",
  "term_label": "mRNA binding",
  "gene": "UniProtKB:O43251",
  "gene_symbol": "RBFOX2"
}